{
  "gene_symbol": "ATP1B3",
  "gene": "UniProtKB:P54709",
  "term_id": "GO:1990573",
  "gene_name": "Sodium_potassium-transporting ATPase subunit beta-3",
  "term_label": "potassium ion import across plasma membrane"
}